{
  "term_label": "positive regulation of cell population proliferation",
  "gene_name": "Vascular endothelial growth factor receptor 2",
  "gene": "UniProtKB:P35968",
  "term_id": "GO:0008284",
  "gene_symbol": "KDR"
}